{
  "gene": "UniProtKB:O00182",
  "gene_name": "Galectin-9",
  "gene_symbol": "LGALS9",
  "term_label": "positive regulation of gene expression",
  "term_id": "GO:0010628"
}